{
  "term_label": "Unknown molecular function",
  "term_id": "UNKNOWN:0001",
  "gene": "UniProtKB:Q4KMZ8",
  "gene_symbol": "NKAIN1",
  "gene_name": "Sodium_potassium-transporting ATPase subunit beta-1-interacting protein 1"
}